{
  "term_id": "GO:0006886",
  "gene": "UniProtKB:Q9H1C4",
  "gene_name": "Protein unc-93 homolog B1",
  "gene_symbol": "UNC93B1",
  "term_label": "intracellular protein transport"
}